symbiont-mediated suppression of host B-cell mediated immune response [GO:0052086] (biological process) Definition: A process by which a symbiont interferes with, inhibits or disrupts the normal execution of the B-cell mediated immune response of the host organism. The host is defined as the larger of the organisms involved in a symbiotic interaction. Sources: GOC:mtg_pamgo_17jul06 Relationships: is a type of symbiont-mediated suppression of host adaptive immune response [GO:0039504] Also known as: negative regulation by organism of B-cell mediated immune response of other organism involved in symbiotic interaction, down regulation by symbiont of host B-cell mediated immune response, down-regulation by symbiont of host B-cell mediated immune response, downregulation by symbiont of host B-cell mediated immune response, suppression by symbiont of host B-cell mediated immune response, suppression of host B-cell mediated immune response, inhibition by symbiont of host B-cell mediated immune response